{
  "gene": "UniProtKB:Q8NAP1",
  "gene_symbol": "CASTOR3P",
  "term_id": "GO:1904262",
  "gene_name": "Putative protein CASTOR3P",
  "term_label": "negative regulation of TORC1 signaling"
}